{
  "gene_symbol": "RNF126",
  "gene": "UniProtKB:Q9BV68",
  "term_label": "cytoplasm",
  "term_id": "GO:0005737",
  "gene_name": "E3 ubiquitin-protein ligase RNF126"
}